farnesyl diphosphatase activity [GO:0120557] (molecular function) Definition: Catalysis of the reaction: (2E,6E)-farnesyl diphosphate + H2O = (2E,6E)-farnesyl phosphate + phosphate + H+. References: PMID:19168029 Sources: RHEA:48128 Relationships: is_a polyprenyl diphosphate phosphatase activity [GO:0120556]